regulation of neurofibrillary tangle assembly [GO:1902996] (biological process) Subtypes: negative regulation of neurofibrillary tangle assembly [GO:1902997], positive regulation of neurofibrillary tangle assembly [GO:1902998] Also known as: regulation of neurofibrillary tangle formation, regulation of flame-shaped neurofibrillary tangle assembly, regulation of flame-shaped neurofibrillary tangle formation, regulation of star-shaped neurofibrillary tangle assembly, regulation of star-shaped neurofibrillary tangle formation Definition: Any process that modulates the frequency, rate or extent of neurofibrillary tangle assembly. Relationships: is a type of regulation of inclusion body assembly [GO:0090083]; regulates GO:1902988 References: PMID:15897157 Sources: GOC:TermGenie, GOC:sjp, GO_REF:0000058